positive regulation of chemokine (C-X-C motif) ligand 9 production [GO:0035396] (biological process) Also known as: positive regulation of CXCL9 production, positive regulation of MIG production Sources: GOC:bf Definition: Any process that activates or increases the frequency, rate, or extent of production of chemokine (C-X-C motif) ligand 9. Relationships: is_a positive regulation of chemokine production [GO:0032722]; is_a regulation of chemokine (C-X-C motif) ligand 9 production [GO:0035394]; positively regulates chemokine (C-X-C motif) ligand 9 production [GO:0035393]